{
  "gene_symbol": "NTSR1",
  "term_id": "GO:0007218",
  "gene_name": "Neurotensin receptor type 1",
  "term_label": "neuropeptide signaling pathway",
  "gene": "UniProtKB:P30989"
}